{
  "term_id": "GO:0005615",
  "gene": "UniProtKB:Q96RP3",
  "gene_name": "Urocortin-2",
  "gene_symbol": "UCN2",
  "term_label": "extracellular space"
}